{
  "term_id": "GO:0005085",
  "gene_name": "PH and SEC7 domain-containing protein 3",
  "term_label": "guanyl-nucleotide exchange factor activity",
  "gene_symbol": "PSD3",
  "gene": "UniProtKB:Q9NYI0"
}